regulation of flavonoid biosynthetic process [GO:0009962] (biological process) Also known as: regulation of flavonoid anabolism, regulation of flavonoid biosynthesis, regulation of flavonoid formation, regulation of flavonoid synthesis Relationships: is a type of regulation of biosynthetic process [GO:0009889]; is a type of regulation of primary metabolic process [GO:0080090]; regulates flavonoid biosynthetic process [GO:0009813] Sources: GOC:tb Subtypes: GO:0009963, GO:0009964, regulation of anthocyanin biosynthetic process [GO:0031540], regulation of flavonol biosynthetic process [GO:1900384] Definition: Any process that modulates the frequency, rate or extent of the chemical reactions and pathways resulting in the formation of flavonoids.